{
  "gene_name": "Dolichol kinase",
  "gene": "UniProtKB:Q9UPQ8",
  "gene_symbol": "DOLK",
  "term_label": "endoplasmic reticulum membrane",
  "term_id": "GO:0005789"
}